centrolateral axis specification [GO:0009947] (biological process) Definition: The establishment, maintenance and elaboration of the centrolateral axis. In plants, this axis is duplicated and runs from the midrib to the margin of the leaf. Sources: GOC:dsz, GOC:tb, ISBN:0865427429 Also known as: mediolateral axis specification, centrolateral axis determination Relationships: is a type of axis specification [GO:0009798]; is part of GO:0097353